midgut development [GO:0007494] (biological process) Relationships: is a type of digestive tract development [GO:0048565] Sources: GOC:jid, UBERON:0001045 Definition: The process whose specific outcome is the progression of the midgut over time, from its formation to the mature structure. The midgut is the middle part of the alimentary canal from the stomach, or entrance of the bile duct, to, or including, the large intestine.